negative regulation of anthocyanin metabolic process [GO:0031538] (biological process) Also known as: down regulation of anthocyanin metabolic process, down-regulation of anthocyanin metabolic process, downregulation of anthocyanin metabolic process, negative regulation of anthocyanin metabolism, inhibition of anthocyanin metabolic process Relationships: is a type of negative regulation of metabolic process [GO:0009892]; is a type of GO:0031537; negatively regulates anthocyanin-containing compound metabolic process [GO:0046283] Definition: Any process that stops, prevents, or reduces the frequency, rate or extent of chemical reactions and pathways involving anthocyanins. Subtypes: GO:0031541, negative regulation of anthocyanin catabolic process [GO:1900001] Sources: GOC:mah